{
  "gene_name": "Putative transmembrane protein INAFM1",
  "gene_symbol": "INAFM1",
  "term_id": "UNKNOWN:0003",
  "gene": "UniProtKB:C9JVW0",
  "term_label": "Unknown cellular component"
}